{
  "term_id": "GO:0090557",
  "gene_symbol": "TJP3",
  "gene": "UniProtKB:O95049",
  "gene_name": "Tight junction protein ZO-3",
  "term_label": "establishment of endothelial intestinal barrier"
}